protein localization to nuclear periphery [GO:1990139] (biological process) Definition: A process in which a protein is transported to, or maintained in, a location within the nuclear periphery. Relationships: is a type of protein localization to nucleus [GO:0034504] References: PMID:23703609 Sources: GOC:mah